mitotic cytokinesis [GO:0000281] (biological process) Also known as: cytokinesis after mitosis Definition: A cell cycle process that results in the division of the cytoplasm of a cell after mitosis, resulting in the separation of the original cell into two daughter cells. Regulation: regulated by GO:1902412; negatively regulated by negative regulation of mitotic cytokinesis [GO:1902413]; positively regulated by positive regulation of mitotic cytokinesis [GO:1903490] Subtypes: zygote asymmetric cytokinesis in embryo sac [GO:0010069] Sources: GOC:mtg_cell_cycle Relationships: is a type of GO:0061640; is_a mitotic cell cycle process [GO:1903047]